{
  "term_label": "basolateral plasma membrane",
  "gene": "UniProtKB:O14936",
  "gene_name": "Peripheral plasma membrane protein CASK",
  "term_id": "GO:0016323",
  "gene_symbol": "CASK"
}